{
  "gene": "UniProtKB:O75995",
  "term_label": "Unknown molecular function",
  "term_id": "UNKNOWN:0001",
  "gene_symbol": "SASH3",
  "gene_name": "SAM and SH3 domain-containing protein 3"
}